chemokine receptor transport out of membrane raft [GO:0032600] (biological process) Relationships: is a type of protein transport out of membrane raft [GO:0032599]; is a type of GO:0033606 Definition: The directed movement of a chemokine receptor out of a membrane raft. Also known as: chemokine receptor translocation out of membrane raft, chemokine receptor transport out of lipid raft Sources: GOC:mah